G-protein gated potassium channel activity [GO:0099101] (molecular function) Definition: A potassium channel activity that is gated by binding of a G-protein beta-gamma dimer. References: PMID:9429760 Sources: GOC:dos Subtypes: GO:0099102 Relationships: is a type of potassium channel activity [GO:0005267]